3' overhang single-stranded DNA endodeoxyribonuclease activity [GO:1990599] (molecular function) References: PMID:25203555 Definition: Catalysis of the hydrolysis of ester linkages within 3' overhang single-stranded deoxyribonucleic acid by creating internal breaks. Relationships: is a type of single-stranded DNA endodeoxyribonuclease activity [GO:0000014]